{
  "gene_name": "Glycoprotein endo-alpha-1,2-mannosidase",
  "gene": "UniProtKB:Q5SRI9",
  "gene_symbol": "MANEA",
  "term_id": "GO:0000139",
  "term_label": "Golgi membrane"
}